{
  "gene_name": "T cell receptor beta constant 1",
  "gene_symbol": "TRBC1",
  "term_id": "UNKNOWN:0002",
  "gene": "UniProtKB:P01850",
  "term_label": "Unknown biological process"
}